CTP-dependent diacylglycerol kinase activity [GO:0141035] (molecular function) Definition: Catalysis of the reaction: a 1,2-diacyl-sn-glycerol + CTP = a 1,2-diacyl-sn-glycero-3-phosphate + CDP + H+. Relationships: is a type of GO:0001727; is a type of GO:0016773 Also known as: DAG kinase activity, diacylglycerol kinase (CTP dependent), diacylglycerol kinase activity, diacylglycerol kinase activity (CTP) Sources: RHEA:25948